triose-phosphate:phosphate antiporter activity [GO:0009670] (molecular function) Definition: Enables the transfer of a solute or solutes from one side of a membrane to the other according to the reaction: triose-phosphate(out) + phosphate(in) = triose-phosphate(in) + phosphate(out). Sources: GOC:bf, GOC:jl, GOC:mtg_transport, ISBN:0815340729, TC:2.A.7.-.- Also known as: dihydroxyacetone phosphate:phosphate antiporter activity, triose phosphate antiporter, triose phosphate translocator, TPT Relationships: is a type of organophosphate:phosphate antiporter activity [GO:0015315]; is a type of GO:0071917 Subtypes: glyceraldehyde 3-phosphate:phosphate antiporter activity [GO:0051408]